10-hydroxy-9-(phosphonooxy)octadecanoate phosphatase activity [GO:0033885] (molecular function) Also known as: dihydroxy fatty acid phosphatase activity, hydroxy fatty acid phosphatase activity, hydroxy lipid phosphatase activity, lipid-phosphate phosphatase activity, (9S,10S)-10-hydroxy-9-(phosphonooxy)octadecanoate phosphohydrolase activity, (9S,10S)-10-hydroxy-9-(phosphonooxy)octadecanoate phosphatase activity, sEH, soluble epoxide hydrolase activity Definition: Catalysis of the reaction: (9S,10S)-10-hydroxy-9-(phosphonooxy)octadecanoate + H2O = (9S,10S)-9,10-dihydroxyoctadecanoate + phosphate. Sources: EC:3.1.3.76, RHEA:16537 Relationships: is a type of phosphatase activity [GO:0016791]